{
  "gene": "UniProtKB:Q9UMR2",
  "gene_name": "ATP-dependent RNA helicase DDX19B",
  "term_label": "cytoplasmic stress granule",
  "term_id": "GO:0010494",
  "gene_symbol": "DDX19B"
}